interleukin-1 type I receptor antagonist activity [GO:0045352] (molecular function) Relationships: is a type of GO:0005152 Also known as: IL-1ra type I Definition: Blocks the binding of interleukin-1 to interleukin-1 type I receptors. Sources: GOC:ebc